{
  "term_id": "GO:1990573",
  "gene_symbol": "ATP4A",
  "gene_name": "Potassium-transporting ATPase alpha chain 1",
  "term_label": "potassium ion import across plasma membrane",
  "gene": "UniProtKB:P20648"
}